{
  "term_label": "Unknown biological process",
  "gene": "UniProtKB:O94952",
  "term_id": "UNKNOWN:0002",
  "gene_name": "F-box only protein 21",
  "gene_symbol": "FBXO21"
}